{
  "gene_name": "Putative beta-lactamase-like 1",
  "gene_symbol": "LACTBL1",
  "term_label": "Unknown cellular component",
  "gene": "UniProtKB:A8MY62",
  "term_id": "UNKNOWN:0003"
}